S-adenosylhomocysteine catabolic process [GO:0019510] (biological process) Relationships: is a type of modified amino acid catabolic process [GO:0042219]; is a type of GO:0044273; is a type of GO:0046130; is a type of GO:0046498; is a type of L-amino acid catabolic process [GO:0170035]; is a type of GO:0170044 Also known as: S-adenosylhomocysteine breakdown, S-adenosylhomocysteine catabolism, S-adenosylhomocysteine degradation Definition: The chemical reactions and pathways resulting in the breakdown of S-adenosylhomocysteine, forming homocysteine and then methionine. Sources: ISBN:0198506732